amoeboid sperm motility [GO:0097723] (biological process) Relationships: is a type of sperm motility [GO:0097722] Definition: Any process involved in the controlled movement of an amoeboid sperm cell. Regulation: regulated by regulation of amoeboid sperm motility [GO:1905416]; negatively regulated by negative regulation of amoeboid sperm motility [GO:1905417]; positively regulated by GO:1905418 Sources: GOC:cilia, GOC:krc Also known as: ameboid sperm motility, ameboid sperm movement, amoeboid sperm movement